distal convoluted tubule development [GO:0072025] (biological process) Relationships: is a type of nephron tubule development [GO:0072080]; is part of distal tubule development [GO:0072017] Sources: GOC:mtg_kidney_jan10 Subtypes: metanephric distal convoluted tubule development [GO:0072221] Definition: The process whose specific outcome is the progression of the distal convoluted tubule over time, from its formation to the mature structure. The distal convoluted tubule is the first segment of the nephron lying just downstream from the loop of Henle, immediately after the macula densa. Among other functions, in humans it is responsible for the reabsorption of about 5% of filtered sodium via the thiazide-sensitive Na-Cl symporter.